{
  "term_id": "GO:0003779",
  "term_label": "actin binding",
  "gene_symbol": "SSH3",
  "gene": "UniProtKB:Q8TE77",
  "gene_name": "Protein phosphatase Slingshot homolog 3"
}